{
  "term_label": "Unknown biological process",
  "gene": "UniProtKB:Q6ZU45",
  "gene_name": "Putative C-type lectin domain family 20 member A",
  "gene_symbol": "CLEC20A",
  "term_id": "UNKNOWN:0002"
}